{
  "gene_name": "Phosphatidylcholine transfer protein",
  "term_label": "phosphatidylcholine binding",
  "gene_symbol": "PCTP",
  "gene": "UniProtKB:Q9UKL6",
  "term_id": "GO:0031210"
}